atrial cardiac muscle tissue morphogenesis [GO:0055009] (biological process) Definition: The process in which the anatomical structure of cardiac atrium muscle is generated and organized. Sources: GOC:devbiol Also known as: atrial heart muscle morphogenesis, atrial myocardium morphogenesis, cardiac atrium muscle morphogenesis Relationships: is a type of cardiac muscle tissue morphogenesis [GO:0055008]; is part of cardiac atrium morphogenesis [GO:0003209]; BFO_0000050 GO:0003228